{
  "gene_name": "cTAGE family member 8",
  "term_label": "endoplasmic reticulum membrane",
  "term_id": "GO:0005789",
  "gene": "UniProtKB:P0CG41",
  "gene_symbol": "CTAGE8"
}